regulation of gliotoxin biosynthetic process [GO:1900689] (biological process) Definition: Any process that modulates the frequency, rate or extent of gliotoxin biosynthetic process. Also known as: regulation of gliotoxin anabolism, regulation of gliotoxin biosynthesis, regulation of gliotoxin formation, regulation of gliotoxin synthesis Relationships: is a type of GO:0034248; is a type of regulation of sulfur metabolic process [GO:0042762]; is a type of GO:1900376; regulates gliotoxin biosynthetic process [GO:2001310] Sources: GOC:TermGenie, GOC:di Subtypes: negative regulation of gliotoxin biosynthetic process [GO:1900690], positive regulation of gliotoxin biosynthetic process [GO:1900691]